N-acylphosphatidylethanolamine metabolic process [GO:0070292] (biological process) Definition: The chemical reactions and pathways involving N-acylphosphatidylethanolamines. An N-acylphosphatidylethanolamine is a phosphatidylethanolamine substituted at nitrogen by an acyl group. Also known as: N-acylphosphatidylethanolamine metabolism, NAPE metabolic process, NAPE metabolism Relationships: is a type of amide metabolic process [GO:0043603]; is a type of phosphatidylethanolamine metabolic process [GO:0046337] References: PMID:14634025, PMID:15878693 Sources: GOC:elh, GOC:mah